{
  "gene_symbol": "CRBN",
  "term_label": "nucleus",
  "gene": "UniProtKB:Q96SW2",
  "term_id": "GO:0005634",
  "gene_name": "Protein cereblon"
}